{
  "term_label": "Unknown cellular component",
  "gene": "UniProtKB:Q14512",
  "term_id": "UNKNOWN:0003",
  "gene_symbol": "FGFBP1",
  "gene_name": "Fibroblast growth factor-binding protein 1"
}